{
  "gene": "UniProtKB:Q96SK3",
  "term_label": "regulation of transcription by RNA polymerase II",
  "gene_name": "Zinc finger protein 607",
  "gene_symbol": "ZNF607",
  "term_id": "GO:0006357"
}